{
  "term_label": "cytoplasm",
  "gene": "UniProtKB:Q9UJC3",
  "term_id": "GO:0005737",
  "gene_symbol": "HOOK1",
  "gene_name": "Protein Hook homolog 1"
}